{
  "gene": "UniProtKB:Q96AZ1",
  "term_id": "UNKNOWN:0002",
  "gene_name": "EEF1A lysine methyltransferase 3",
  "gene_symbol": "EEF1AKMT3",
  "term_label": "Unknown biological process"
}